{
  "gene": "UniProtKB:Q15262",
  "gene_symbol": "PTPRK",
  "gene_name": "Receptor-type tyrosine-protein phosphatase kappa",
  "term_id": "GO:0004725",
  "term_label": "protein tyrosine phosphatase activity"
}